{
  "term_id": "GO:0045022",
  "gene_symbol": "PTPN23",
  "gene": "UniProtKB:Q9H3S7",
  "gene_name": "Tyrosine-protein phosphatase non-receptor type 23",
  "term_label": "early endosome to late endosome transport"
}